{
  "term_id": "GO:0034450",
  "gene_name": "RING finger protein 37",
  "gene": "UniProtKB:O94941",
  "gene_symbol": "UBOX5",
  "term_label": "ubiquitin-ubiquitin ligase activity"
}